NADPH oxidase complex [GO:0043020] (cellular component) Also known as: flavocytochrome b558, respiratory-burst oxidase Relationships: is a type of plasma membrane protein complex [GO:0098797]; is a type of GO:1990204 Definition: A enzyme complex of which the core is a heterodimer composed of a light (alpha) and heavy (beta) chain, and requires the cytosolic regulatory subunits at least NCF1/p47-phox, NCF2/p67-phox, NCF4/p40-phox and the small GTPase RAC1 or RAC2 for activity. Functions in superoxide generation by the NADPH-dependent reduction of O2. References: PMID:11483596, PMID:12440767 Sources: GOC:jl